{
  "term_id": "GO:0070765",
  "gene_symbol": "APH1B",
  "gene": "UniProtKB:Q8WW43",
  "term_label": "gamma-secretase complex",
  "gene_name": "Gamma-secretase subunit APH-1B"
}